{
  "gene_symbol": "MRPS16",
  "gene": "UniProtKB:Q9Y3D3",
  "term_label": "mitochondrial small ribosomal subunit",
  "gene_name": "Small ribosomal subunit protein bS16m",
  "term_id": "GO:0005763"
}